{
  "gene_name": "Apelin receptor early endogenous ligand",
  "gene": "UniProtKB:P0DMC3",
  "term_id": "GO:0005576",
  "term_label": "extracellular region",
  "gene_symbol": "APELA"
}